{
  "term_id": "UNKNOWN:0001",
  "term_label": "Unknown molecular function",
  "gene": "UniProtKB:P56597",
  "gene_name": "Nucleoside diphosphate kinase homolog 5",
  "gene_symbol": "NME5"
}